{
  "gene_symbol": "ACSM1",
  "term_id": "GO:0004321",
  "gene_name": "Acyl-coenzyme A synthetase ACSM1, mitochondrial",
  "gene": "UniProtKB:Q08AH1",
  "term_label": "fatty-acyl-CoA synthase activity"
}